{
  "gene_name": "Putative testis-specific prion protein",
  "gene": "UniProtKB:Q86SH4",
  "gene_symbol": "PRNT",
  "term_label": "Unknown biological process",
  "term_id": "UNKNOWN:0002"
}